{
  "gene": "UniProtKB:Q8NHU3",
  "term_label": "ceramide cholinephosphotransferase activity",
  "gene_name": "Phosphatidylcholine:ceramide cholinephosphotransferase 2",
  "gene_symbol": "SGMS2",
  "term_id": "GO:0047493"
}